negative regulation of corticotropin-releasing hormone secretion [GO:0051465] (biological process) Also known as: down regulation of corticotropin-releasing hormone secretion, down-regulation of corticotropin-releasing hormone secretion, downregulation of corticotropin-releasing hormone secretion, negative regulation of CRF secretion, negative regulation of CRH secretion, negative regulation of corticotropin-releasing factor secretion, inhibition of corticotropin-releasing hormone secretion Relationships: is a type of GO:0043397; is a type of GO:0090278; negatively regulates corticotropin-releasing hormone secretion [GO:0043396] Definition: Any process that stops, prevents, or reduces the frequency, rate or extent of the regulated release of corticotropin-releasing hormone from a cell. Sources: GOC:ai